cellopentaose binding [GO:0044587] (molecular function) Definition: Binding to a cellopentaose, an oligosaccharide consisting of four glucose residues resulting from hydrolysis of cellulose. Relationships: is a type of oligosaccharide binding [GO:0070492] Sources: GOC:mengo_curators, GOC:tt